{
  "gene": "UniProtKB:Q92874",
  "term_id": "GO:0004530",
  "gene_name": "Deoxyribonuclease-1-like 2",
  "gene_symbol": "DNASE1L2",
  "term_label": "deoxyribonuclease I activity"
}